uridylyltransferase activity [GO:0070569] (molecular function) Also known as: uridyl transferase activity, uridyltransferase activity Definition: Catalysis of the transfer of an uridylyl group to an acceptor. Relationships: is a type of nucleotidyltransferase activity [GO:0016779] Sources: GOC:mah Subtypes: UDP-N-acetylglucosamine diphosphorylase activity [GO:0003977], UDP-glucose:hexose-1-phosphate uridylyltransferase activity [GO:0008108], [protein-PII] uridylyltransferase activity [GO:0008773], glucuronate-1-phosphate uridylyltransferase activity [GO:0047350], RNA uridylyltransferase activity [GO:0050265], UTP-monosaccharide-1-phosphate uridylyltransferase activity [GO:0051748], UDP-N-acetylgalactosamine diphosphorylase activity [GO:0052630]